{
  "term_label": "extracellular space",
  "gene_symbol": "IGFBP6",
  "term_id": "GO:0005615",
  "gene_name": "Insulin-like growth factor-binding protein 6",
  "gene": "UniProtKB:P24592"
}